{
  "term_label": "Unknown biological process",
  "gene_name": "Zinc finger protein 804A",
  "gene_symbol": "ZNF804A",
  "gene": "UniProtKB:Q7Z570",
  "term_id": "UNKNOWN:0002"
}